{
  "gene_symbol": "PROX1",
  "term_label": "nucleus",
  "gene_name": "Prospero homeobox protein 1",
  "term_id": "GO:0005634",
  "gene": "UniProtKB:Q92786"
}